chloride peroxidase activity [GO:0016691] (molecular function) Definition: Catalysis of the reaction: 2 R-H + 2 chloride + H2O2 = 2 R-Cl + 2 H2O. Also known as: cofactor-free chloroperoxidase activity, flavin-haem chloroperoxidase activity, flavin-heme chloroperoxidase activity, haem chloroperoxidase activity, heme chloroperoxidase activity, vanadium chloroperoxidase activity, chloride:hydrogen-peroxide oxidoreductase, chloroperoxidase activity Relationships: is a type of haloperoxidase activity [GO:0140905] Sources: EC:1.11.1.10